{
  "term_id": "GO:0030258",
  "gene_symbol": "MBOAT7",
  "gene_name": "Lysophospholipid acyltransferase 7",
  "term_label": "lipid modification",
  "gene": "UniProtKB:Q96N66"
}